{
  "gene_name": "Protocadherin alpha-1",
  "gene_symbol": "PCDHA1",
  "gene": "UniProtKB:Q9Y5I3",
  "term_label": "cell adhesion",
  "term_id": "GO:0007155"
}